{
  "term_label": "regulation of transcription by RNA polymerase II",
  "gene_name": "Heart- and neural crest derivatives-expressed protein 1",
  "gene": "UniProtKB:O96004",
  "term_id": "GO:0006357",
  "gene_symbol": "HAND1"
}